{
  "term_id": "GO:0001578",
  "gene_symbol": "MTCL1",
  "gene": "UniProtKB:Q9Y4B5",
  "gene_name": "Microtubule cross-linking factor 1",
  "term_label": "microtubule bundle formation"
}